{
  "term_label": "cell fate commitment",
  "gene": "UniProtKB:P56705",
  "gene_name": "Protein Wnt-4",
  "term_id": "GO:0045165",
  "gene_symbol": "WNT4"
}